{
  "gene_symbol": "CCK",
  "gene_name": "Cholecystokinin",
  "term_label": "digestion",
  "gene": "UniProtKB:P06307",
  "term_id": "GO:0007586"
}